{
  "term_id": "UNKNOWN:0002",
  "gene_symbol": "IER2",
  "gene": "UniProtKB:Q9BTL4",
  "gene_name": "Immediate early response gene 2 protein",
  "term_label": "Unknown biological process"
}